{
  "gene_name": "Surfeit locus protein 6",
  "gene": "UniProtKB:O75683",
  "gene_symbol": "SURF6",
  "term_id": "GO:0003677",
  "term_label": "DNA binding"
}